clathrin coat of endocytic vesicle [GO:0030128] (cellular component) Also known as: clathrin coat of endocytotic vesicle Definition: A clathrin coat found on an endocytic vesicle. Relationships: is a type of GO:0030125; is part of GO:0030669 Sources: GOC:mah